{
  "gene": "UniProtKB:P12319",
  "gene_name": "High affinity immunoglobulin epsilon receptor subunit alpha",
  "term_label": "cell surface receptor signaling pathway",
  "term_id": "GO:0007166",
  "gene_symbol": "FCER1A"
}